{
  "gene": "UniProtKB:P05538",
  "gene_symbol": "HLA-DQB2",
  "term_label": "peptide antigen assembly with MHC class II protein complex",
  "term_id": "GO:0002503",
  "gene_name": "HLA class II histocompatibility antigen, DQ beta 2 chain"
}